{
  "term_id": "GO:0007156",
  "gene_symbol": "CLSTN1",
  "gene": "UniProtKB:O94985",
  "term_label": "homophilic cell-cell adhesion",
  "gene_name": "Calsyntenin-1"
}